spliceosome conformational change to release U4 (or U4atac) and U1 (or U11) [GO:0000388] (BP) Also known as: 3'-splice site cleavage, exon ligation, U12-type spliceosome conformational change to release U4atac and U11, U2-type spliceosome conformational change to release U4 and U1, spliceosomal A1 complex biosynthesis, spliceosomal A1 complex formation, spliceosomal B2 complex biosynthesis, spliceosomal B2 complex formation Relationships: is_a GO:0022618; is part of GO:0000393 Definition: Rearrangement of the pre-catalytic spliceosome containing U4 (or U4atac) and U1 (or U11) snRNPs to unpair U4 (or U4atac) from U6 (or U6atac) and release it from the spliceosomal complex along with U1 (or U11). Sources: GOC:krc, ISBN:0879695897 Note: Note that this step represents formation of the A1 complex (yeast) or the B2 complex (mammalian).